attachment organelle [GO:0033099] (cellular component) Relationships: is a type of intracellular membrane-bounded organelle [GO:0043231] Definition: A membrane-bounded extension of the cell, originally characterized in Mycoplasma species, that contains an electron-dense core that is part of the cytoskeleton and is oriented lengthwise and ends distally in a bulbous knob (terminal button). Required for adherence to host cells and involved in gliding motility and cell division. References: PMID:11325545, PMID:12003948